{
  "term_label": "axon guidance",
  "term_id": "GO:0007411",
  "gene_name": "Semaphorin-6C",
  "gene_symbol": "SEMA6C",
  "gene": "UniProtKB:Q9H3T2"
}